{
  "term_id": "UNKNOWN:0002",
  "term_label": "Unknown biological process",
  "gene": "UniProtKB:P46020",
  "gene_symbol": "PHKA1",
  "gene_name": "Phosphorylase b kinase regulatory subunit alpha, skeletal muscle isoform"
}